positive regulation of ferricrocin biosynthetic process [GO:1900680] (biological process) Relationships: is a type of regulation of ferricrocin biosynthetic process [GO:1900678]; is a type of GO:1905570; positively regulates ferricrocin biosynthetic process [GO:0031171] Also known as: activation of ferricrocin anabolism, activation of ferricrocin biosynthesis, activation of ferricrocin formation, activation of ferricrocin synthesis, positive regulation of ferricrocin anabolism, positive regulation of ferricrocin biosynthesis, positive regulation of ferricrocin formation, positive regulation of ferricrocin synthesis, up regulation of ferricrocin anabolism, up regulation of ferricrocin biosynthesis, up regulation of ferricrocin biosynthetic process, up regulation of ferricrocin formation, up regulation of ferricrocin synthesis, up-regulation of ferricrocin anabolism, up-regulation of ferricrocin biosynthesis, up-regulation of ferricrocin biosynthetic process, up-regulation of ferricrocin formation, up-regulation of ferricrocin synthesis, upregulation of ferricrocin anabolism, upregulation of ferricrocin biosynthesis, upregulation of ferricrocin biosynthetic process, upregulation of ferricrocin formation, upregulation of ferricrocin synthesis, activation of ferricrocin biosynthetic process, activation of ferricrocin biosynthetic process, peptide formation, activation of ferricrocin biosynthetic process, peptide modification, positive regulation of ferricrocin biosynthetic process, peptide formation, positive regulation of ferricrocin biosynthetic process, peptide modification, up regulation of ferricrocin biosynthetic process, peptide formation, up regulation of ferricrocin biosynthetic process, peptide modification, up-regulation of ferricrocin biosynthetic process, peptide formation, up-regulation of ferricrocin biosynthetic process, peptide modification, upregulation of ferricrocin biosynthetic process, peptide formation, upregulation of ferricrocin biosynthetic process, peptide modification Sources: GOC:TermGenie, GOC:di Definition: Any process that activates or increases the frequency, rate or extent of ferricrocin biosynthetic process.